{
  "gene_symbol": "SRRM2",
  "gene": "UniProtKB:Q9UQ35",
  "term_id": "GO:0003729",
  "term_label": "mRNA binding",
  "gene_name": "Serine_arginine repetitive matrix protein 2"
}